long-day photoperiodism [GO:0048571] (biological process) Also known as: response to long-day, response to short-night, short-night photoperiodism, response to long-day photoperiod Subtypes: long-day photoperiodism, flowering [GO:0048574] Definition: Any process that results in a change in state or activity of an organism (in terms of movement, secretion, enzyme production, gene expression, etc.) as a result of detection of, or exposure to, a day length that exceeds a particular duration known as the 'critical day length'. The critical day length varies between species. Although the term long-day is used, most species actually respond to the duration of the night, so that the response will occur when a period of darkness falls short of the number of hours defined by 24 hours minus the critical day length. Relationships: is a type of photoperiodism [GO:0009648] Sources: GOC:jid, GOC:pj, ISBN:0582015952, ISBN:0697037754, ISBN:0709408862